{
  "gene_symbol": "TRIM49C",
  "gene": "UniProtKB:P0CI26",
  "term_id": "GO:0045087",
  "term_label": "innate immune response",
  "gene_name": "Tripartite motif-containing protein 49C"
}